{
  "term_label": "mitochondrion",
  "gene_name": "Bifunctional methylenetetrahydrofolate dehydrogenase_cyclohydrolase, mitochondrial",
  "term_id": "GO:0005739",
  "gene": "UniProtKB:P13995",
  "gene_symbol": "MTHFD2"
}